{
  "gene_name": "Zinc-regulated GTPase metalloprotein activator 1B",
  "gene": "UniProtKB:Q8IUF1",
  "term_id": "GO:0140827",
  "gene_symbol": "ZNG1B",
  "term_label": "zinc chaperone activity"
}